{
  "term_label": "cell adhesion",
  "gene_name": "Sialic acid-binding Ig-like lectin 9",
  "gene_symbol": "SIGLEC9",
  "term_id": "GO:0007155",
  "gene": "UniProtKB:Q9Y336"
}